isobutanol biosynthetic process [GO:1901961] (biological process) Also known as: isobutanol anabolism, isobutanol biosynthesis, isobutanol formation, isobutanol synthesis References: PMID:22224870 Sources: GOC:TermGenie, GOC:mengo_curators Relationships: is a type of primary alcohol biosynthetic process [GO:0034309] Definition: The chemical reactions and pathways resulting in the formation of isobutanol.